{
  "gene_name": "Lipopolysaccharide-responsive and beige-like anchor protein",
  "term_label": "protein kinase binding",
  "gene": "UniProtKB:P50851",
  "term_id": "GO:0019901",
  "gene_symbol": "LRBA"
}